{
  "gene_symbol": "DLX6",
  "term_label": "RNA polymerase II cis-regulatory region sequence-specific DNA binding",
  "gene": "UniProtKB:P56179",
  "gene_name": "Homeobox protein DLX-6",
  "term_id": "GO:0000978"
}